{
  "term_id": "GO:0019901",
  "gene": "UniProtKB:Q8TDY2",
  "term_label": "protein kinase binding",
  "gene_name": "RB1-inducible coiled-coil protein 1",
  "gene_symbol": "RB1CC1"
}